positive regulation of purine nucleotide biosynthetic process [GO:1900373] (biological process) Subtypes: positive regulation of guanylate cyclase activity [GO:0031284], positive regulation of 'de novo' NAD biosynthetic process from L-tryptophan [GO:1905014], positive regulation of ATP biosynthetic process [GO:2001171] Relationships: is a type of positive regulation of nucleotide biosynthetic process [GO:0030810]; is a type of regulation of purine nucleotide biosynthetic process [GO:1900371]; is a type of GO:1900544; positively regulates purine nucleotide biosynthetic process [GO:0006164] Definition: Any process that activates or increases the frequency, rate or extent of purine nucleotide biosynthetic processes. Also known as: activation of purine nucleotide anabolism, activation of purine nucleotide biosynthesis, activation of purine nucleotide formation, activation of purine nucleotide synthesis, positive regulation of purine nucleotide anabolism, positive regulation of purine nucleotide biosynthesis, positive regulation of purine nucleotide formation, positive regulation of purine nucleotide synthesis, up regulation of purine nucleotide anabolism, up regulation of purine nucleotide biosynthesis, up regulation of purine nucleotide biosynthetic process, up regulation of purine nucleotide formation, up regulation of purine nucleotide synthesis, up-regulation of purine nucleotide anabolism, up-regulation of purine nucleotide biosynthesis, up-regulation of purine nucleotide biosynthetic process, up-regulation of purine nucleotide formation, up-regulation of purine nucleotide synthesis, upregulation of purine nucleotide anabolism, upregulation of purine nucleotide biosynthesis, upregulation of purine nucleotide biosynthetic process, upregulation of purine nucleotide formation, upregulation of purine nucleotide synthesis, activation of purine nucleotide biosynthetic process Sources: GOC:TermGenie, GOC:go_curators